maintenance of vegetative meristem identity [GO:0010079] (biological process) Definition: The process in which an organism retains a population of vegetative meristem cells, preventing the commitment of all stem cell progeny to a differentiated cell fate. Relationships: is a type of maintenance of meristem identity [GO:0010074] Sources: GOC:dph, GOC:tb